{
  "term_id": "GO:0032435",
  "gene_name": "NEDD4-binding protein 1",
  "gene_symbol": "N4BP1",
  "gene": "UniProtKB:O75113",
  "term_label": "negative regulation of proteasomal ubiquitin-dependent protein catabolic process"
}